{
  "gene_name": "Teratocarcinoma-derived growth factor 1",
  "gene_symbol": "TDGF1",
  "term_label": "activin receptor binding",
  "term_id": "GO:0070697",
  "gene": "UniProtKB:P13385"
}